positive regulation of intrinsic apoptotic signaling pathway [GO:2001244] (biological process) Subtypes: positive regulation of oxidative stress-induced intrinsic apoptotic signaling pathway [GO:1902177], positive regulation of intrinsic apoptotic signaling pathway in response to osmotic stress [GO:1902220], positive regulation of intrinsic apoptotic signaling pathway in response to DNA damage [GO:1902231], positive regulation of endoplasmic reticulum stress-induced intrinsic apoptotic signaling pathway [GO:1902237], positive regulation of intrinsic apoptotic signaling pathway by p53 class mediator [GO:1902255], positive regulation of nitrosative stress-induced intrinsic apoptotic signaling pathway [GO:1905260] Definition: Any process that activates or increases the frequency, rate or extent of intrinsic apoptotic signaling pathway. Relationships: is_a GO:1902533; is a type of positive regulation of apoptotic signaling pathway [GO:2001235]; is a type of GO:2001242; positively regulates GO:0097193 Sources: GOC:mtg_apoptosis Also known as: positive regulation of intrinsic apoptotic pathway, positive regulation of intrinsic apoptotic signalling pathway, positive regulation of mitochondrial-mediated apoptotic pathway, positive regulation of intrinsic apoptosis